retinoic acid binding [GO:0001972] (molecular function) Relationships: is a type of retinoid binding [GO:0005501]; is a type of monocarboxylic acid binding [GO:0033293] Definition: Binding to retinoic acid, 3,7-dimethyl-9-(2,6,-trimethyl-1-cyclohexen-1-yl)-2,4,6,8-nonatetraenoic acid. Sources: GOC:hjd